{
  "term_label": "cell surface receptor signaling pathway",
  "gene_name": "Probable non-functional T cell receptor beta variable 7-3",
  "gene": "UniProtKB:A0A075B6L6",
  "term_id": "GO:0007166",
  "gene_symbol": "TRBV7-3"
}